{
  "gene_symbol": "SYNM",
  "term_id": "GO:0017166",
  "gene": "UniProtKB:O15061",
  "gene_name": "Synemin",
  "term_label": "vinculin binding"
}